{
  "gene_name": "Ras-related protein Rab-8B",
  "gene": "UniProtKB:Q92930",
  "term_id": "GO:0003924",
  "gene_symbol": "RAB8B",
  "term_label": "GTPase activity"
}